{
  "gene": "UniProtKB:Q96C01",
  "gene_name": "Protein FAM136A",
  "term_label": "Unknown biological process",
  "term_id": "UNKNOWN:0002",
  "gene_symbol": "FAM136A"
}